{
  "gene": "UniProtKB:Q9UPY6",
  "term_id": "GO:0071933",
  "gene_name": "Actin-binding protein WASF3",
  "term_label": "Arp2/3 complex binding",
  "gene_symbol": "WASF3"
}